{
  "term_label": "gluconeogenesis",
  "gene_name": "Pyruvate carboxylase, mitochondrial",
  "gene_symbol": "PC",
  "term_id": "GO:0006094",
  "gene": "UniProtKB:P11498"
}